{
  "term_id": "UNKNOWN:0003",
  "gene_name": "F-box only protein 7",
  "gene_symbol": "FBXO7",
  "gene": "UniProtKB:Q9Y3I1",
  "term_label": "Unknown cellular component"
}